{
  "term_id": "GO:0006413",
  "term_label": "translational initiation",
  "gene_name": "ATP-binding cassette sub-family E member 1",
  "gene": "UniProtKB:P61221",
  "gene_symbol": "ABCE1"
}